dendritic cell cytokine production [GO:0002371] (biological process) Subtypes: myeloid dendritic cell cytokine production [GO:0002372], plasmacytoid dendritic cell cytokine production [GO:0002373] Sources: GOC:add, ISBN:0781735149 Note: Note that this term is in the subset of terms that should not be used for direct gene product annotation. Instead, select one of the 'regulation' children terms. Relationships: is a type of cytokine production involved in immune response [GO:0002367]; is a type of GO:0002443 Definition: Any process that contributes to cytokine production by a dendritic cell. Regulation: regulated by regulation of dendritic cell cytokine production [GO:0002730]; negatively regulated by negative regulation of dendritic cell cytokine production [GO:0002731]; RO_0002213 by GO:0002732